{
  "term_label": "regulation of protein localization to plasma membrane",
  "gene": "UniProtKB:Q13555",
  "gene_symbol": "CAMK2G",
  "gene_name": "Calcium_calmodulin-dependent protein kinase type II subunit gamma",
  "term_id": "GO:1903076"
}